quercetin 4'-O-glucosyltransferase activity [GO:0080046] (molecular function) Relationships: is a type of UDP-glucosyltransferase activity [GO:0035251] References: PMID:15352060 Definition: Catalysis of the transfer of a glucosyl group from UDP-glucose to the 4'-hydroxy group of a quercetin molecule.